{
  "gene": "UniProtKB:P51857",
  "term_label": "aldose reductase (NADPH) activity",
  "gene_symbol": "AKR1D1",
  "term_id": "GO:0004032",
  "gene_name": "Aldo-keto reductase family 1 member D1"
}